{
  "term_label": "intracellular protein localization",
  "gene": "UniProtKB:Q9BXJ7",
  "term_id": "GO:0008104",
  "gene_name": "Protein amnionless",
  "gene_symbol": "AMN"
}